{
  "gene_name": "Fanconi anemia group A protein",
  "gene": "UniProtKB:O15360",
  "term_id": "UNKNOWN:0001",
  "term_label": "Unknown molecular function",
  "gene_symbol": "FANCA"
}